{
  "gene_symbol": "NAAA",
  "gene": "UniProtKB:Q02083",
  "term_label": "Unknown cellular component",
  "term_id": "UNKNOWN:0003",
  "gene_name": "N-acylethanolamine-hydrolyzing acid amidase"
}